{
  "term_id": "GO:0000122",
  "gene": "UniProtKB:P48436",
  "term_label": "negative regulation of transcription by RNA polymerase II",
  "gene_symbol": "SOX9",
  "gene_name": "Transcription factor SOX-9"
}